{
  "gene_symbol": "SFT2D2",
  "term_id": "UNKNOWN:0002",
  "gene_name": "Vesicle transport protein SFT2B",
  "term_label": "Unknown biological process",
  "gene": "UniProtKB:O95562"
}